{
  "gene": "UniProtKB:Q8IVP5",
  "term_id": "GO:0005741",
  "gene_name": "FUN14 domain-containing protein 1",
  "term_label": "mitochondrial outer membrane",
  "gene_symbol": "FUNDC1"
}